apoptotic process involved in development [GO:1902742] (biological process) Definition: Any apoptotic process that is involved in anatomical structure development. Sources: GOC:TermGenie, GOC:mtg_apoptosis, GOC:pg, GO_REF:0000060 Also known as: apoptotic cell death involved in anatomical structure development, apoptotic cell death involved in development of an anatomical structure, apoptotic process involved in anatomical structure development, apoptotic process involved in development of an anatomical structure, apoptotic programmed cell death involved in anatomical structure development, apoptotic programmed cell death involved in development of an anatomical structure, programmed cell death by apoptosis involved in anatomical structure development, programmed cell death by apoptosis involved in development of an anatomical structure, activation of apoptosis involved in anatomical structure development, activation of apoptosis involved in development of an anatomical structure, apoptosis involved in anatomical structure development, apoptosis involved in development of an anatomical structure, apoptosis signaling involved in anatomical structure development, apoptosis signaling involved in development of an anatomical structure, apoptotic program involved in anatomical structure development, apoptotic program involved in development of an anatomical structure, type I programmed cell death involved in anatomical structure development, type I programmed cell death involved in development of an anatomical structure, apoptosis activator activity involved in anatomical structure development, apoptosis activator activity involved in development of an anatomical structure, commitment to apoptosis involved in anatomical structure development, commitment to apoptosis involved in development of an anatomical structure, induction of apoptosis by p53 involved in anatomical structure development, induction of apoptosis by p53 involved in development of an anatomical structure, induction of apoptosis involved in anatomical structure development, induction of apoptosis involved in development of an anatomical structure, signaling (initiator) caspase activity involved in anatomical structure development, signaling (initiator) caspase activity involved in development of an anatomical structure Relationships: is_a GO:0006915; is part of anatomical structure development [GO:0048856] Subtypes: B cell deletion [GO:0002516], nurse cell apoptotic process [GO:0045476], apoptotic process involved in morphogenesis [GO:0060561], apoptotic process involved in luteolysis [GO:0061364], mesenchymal cell apoptotic process involved in metanephros development [GO:1900200], apoptotic process involved in metanephric collecting duct development [GO:1900204], apoptotic process involved in metanephric nephron tubule development [GO:1900205] Regulation: RO_0002212 by negative regulation of apoptotic process involved in development [GO:1904746]; positively regulated by positive regulation of apoptotic process involved in development [GO:1904747]; regulated by regulation of apoptotic process involved in development [GO:1904748]